{
  "gene": "UniProtKB:Q6UX39",
  "term_id": "UNKNOWN:0001",
  "term_label": "Unknown molecular function",
  "gene_symbol": "AMTN",
  "gene_name": "Amelotin"
}